embryonic hindgut morphogenesis [GO:0048619] (biological process) Definition: The process in which the anatomical structures of the hindgut are generated and organized, during the embryonic phase. Sources: GOC:jid, GOC:rc Relationships: is a type of GO:0048598; is part of hindgut morphogenesis [GO:0007442]